{
  "term_id": "UNKNOWN:0001",
  "gene_name": "LYR motif-containing protein 2",
  "gene_symbol": "LYRM2",
  "gene": "UniProtKB:Q9NU23",
  "term_label": "Unknown molecular function"
}